{
  "gene_symbol": "ERGIC2",
  "term_label": "COPII-coated ER to Golgi transport vesicle",
  "gene_name": "Endoplasmic reticulum-Golgi intermediate compartment protein 2",
  "gene": "UniProtKB:Q96RQ1",
  "term_id": "GO:0030134"
}